{
  "term_label": "embryonic skeletal system morphogenesis",
  "term_id": "GO:0048704",
  "gene": "UniProtKB:P31269",
  "gene_name": "Homeobox protein Hox-A9",
  "gene_symbol": "HOXA9"
}